process utilizing autophagic mechanism [GO:0061919] (biological process) Relationships: is a type of cellular process [GO:0009987] Definition: A cellular process involving delivery of a portion of the cytoplasm to lysosomes or to the plant or fungal vacuole that does not involve direct transport through the endocytic or vacuolar protein sorting (Vps) pathways. This process typically leads to degradation of the cargo; however, it can also be used to deliver resident proteins, such as in the cytoplasm-to-vacuole targeting (Cvt) pathway. References: PMID:21997368, PMID:22966490, PMID:28596378 Subtypes: GO:0006914, cytoplasm to vacuole targeting by the Cvt pathway [GO:0032258]